double membrane vesicle viral factory outer membrane [GO:0062243] (cellular component) Definition: The outer of the two endoplasmic reticulum-derived lipid bilayer membranes that bound a double membrane vesicle viral factory. Relationships: is a type of double membrane vesicle viral factory membrane [GO:0062242] References: PMID:22440839 Also known as: outer membrane of double membrane vesicle viral factory